intramolecular oxidoreductase activity [GO:0016860] (molecular function) Definition: Catalysis of an oxidation-reduction (redox) reaction in which the hydrogen donor and acceptor are the same molecule, and no oxidized product appears. Sources: EC:5.3.-.-, GOC:curators Subtypes: prostaglandin-D synthase activity [GO:0004667], thromboxane-A synthase activity [GO:0004796], prostaglandin-I synthase activity [GO:0008116], GO:0016861, intramolecular oxidoreductase activity, interconverting keto- and enol-groups [GO:0016862], GO:0016863, intramolecular oxidoreductase activity, transposing S-S bonds [GO:0016864], GO:0018845, styrene-oxide isomerase activity [GO:0018846], GO:0034020, lycopene epsilon cyclase activity [GO:0045435], lycopene beta cyclase activity [GO:0045436], allene-oxide cyclase activity [GO:0046423], GO:0050220, capsanthin synthase activity [GO:0052727], capsorubin synthase activity [GO:0052728] Relationships: is a type of isomerase activity [GO:0016853] Also known as: intramolecular isomerase activity, intramolecular oxidoreductase activity, other intramolecular oxidoreductases